{
  "gene_symbol": "TOMM22",
  "term_id": "GO:0008320",
  "gene": "UniProtKB:Q9NS69",
  "term_label": "protein transmembrane transporter activity",
  "gene_name": "Mitochondrial import receptor subunit TOM22 homolog"
}